{
  "gene_name": "Solute carrier family 35 member G1",
  "term_label": "endoplasmic reticulum membrane",
  "gene": "UniProtKB:Q2M3R5",
  "gene_symbol": "SLC35G1",
  "term_id": "GO:0005789"
}